{
  "gene_symbol": "LBR",
  "term_label": "nuclear inner membrane",
  "gene": "UniProtKB:Q14739",
  "term_id": "GO:0005637",
  "gene_name": "Delta(14)-sterol reductase LBR"
}